{
  "term_id": "UNKNOWN:0001",
  "gene": "UniProtKB:A7MCY6",
  "term_label": "Unknown molecular function",
  "gene_symbol": "TBKBP1",
  "gene_name": "TANK-binding kinase 1-binding protein 1"
}